{
  "term_id": "GO:0005041",
  "gene": "UniProtKB:P01130",
  "term_label": "low-density lipoprotein particle receptor activity",
  "gene_name": "Low-density lipoprotein receptor",
  "gene_symbol": "LDLR"
}